{
  "term_id": "GO:0005637",
  "gene_name": "Transmembrane protein 120B",
  "gene": "UniProtKB:A0PK00",
  "gene_symbol": "TMEM120B",
  "term_label": "nuclear inner membrane"
}